{
  "gene": "UniProtKB:Q8NB14",
  "term_label": "cytosol",
  "gene_symbol": "USP38",
  "term_id": "GO:0005829",
  "gene_name": "Ubiquitin carboxyl-terminal hydrolase 38"
}